{
  "gene_name": "Stress-associated endoplasmic reticulum protein 1",
  "gene_symbol": "SERP1",
  "term_label": "endoplasmic reticulum",
  "gene": "UniProtKB:Q9Y6X1",
  "term_id": "GO:0005783"
}